{
  "gene_symbol": "ATPSCKMT",
  "gene": "UniProtKB:Q6P4H8",
  "term_id": "GO:0005739",
  "term_label": "mitochondrion",
  "gene_name": "ATP synthase subunit C lysine N-methyltransferase"
}